{
  "term_label": "innate immune response",
  "gene_name": "Putative tripartite motif-containing protein 61",
  "gene": "UniProtKB:Q5EBN2",
  "gene_symbol": "TRIM61",
  "term_id": "GO:0045087"
}